{
  "gene": "UniProtKB:Q14676",
  "term_label": "DNA replication checkpoint signaling",
  "gene_name": "Mediator of DNA damage checkpoint protein 1",
  "term_id": "GO:0000076",
  "gene_symbol": "MDC1"
}